{
  "term_id": "GO:0006298",
  "gene": "UniProtKB:P43246",
  "gene_name": "DNA mismatch repair protein Msh2",
  "gene_symbol": "MSH2",
  "term_label": "mismatch repair"
}